{
  "gene": "UniProtKB:A0A075B6Z9",
  "gene_symbol": "TRAJ24",
  "term_label": "Unknown molecular function",
  "term_id": "UNKNOWN:0001",
  "gene_name": "T cell receptor alpha joining 24 (Fragment)"
}